{
  "term_label": "cytoplasm",
  "term_id": "GO:0005737",
  "gene_symbol": "PVALB",
  "gene_name": "Parvalbumin alpha",
  "gene": "UniProtKB:P20472"
}